{
  "gene_symbol": "C3AR1",
  "gene": "UniProtKB:Q16581",
  "gene_name": "C3a anaphylatoxin chemotactic receptor",
  "term_id": "GO:0007200",
  "term_label": "phospholipase C-activating G protein-coupled receptor signaling pathway"
}